{
  "gene": "UniProtKB:Q99719",
  "term_label": "GTPase activity",
  "gene_name": "Septin-5",
  "term_id": "GO:0003924",
  "gene_symbol": "SEPTIN5"
}